{
  "gene_name": "START domain-containing protein 10",
  "term_id": "UNKNOWN:0001",
  "term_label": "Unknown molecular function",
  "gene": "UniProtKB:Q9Y365",
  "gene_symbol": "STARD10"
}